glucose 1-phosphate phosphorylation [GO:0006009] (biological process) Definition: The process of introducing a phosphate group into glucose 1-phosphate to produce glucose bisphosphate. Relationships: is a type of phosphorylation [GO:0016310]; is a type of glucose 1-phosphate metabolic process [GO:0019255] Sources: GOC:ai